positive regulation of mitotic recombination [GO:0045951] (biological process) Also known as: up regulation of mitotic recombination, up-regulation of mitotic recombination, upregulation of mitotic recombination, activation of mitotic recombination, positive regulation of recombination within rDNA repeats, stimulation of mitotic recombination Definition: Any process that activates or increases the frequency, rate or extent of DNA recombination during mitosis. Sources: GOC:go_curators Subtypes: GO:0032209 Relationships: is a type of regulation of mitotic recombination [GO:0000019]; is a type of GO:0045911; positively regulates mitotic recombination [GO:0006312]